negative regulation of neutrophil mediated killing of bacterium [GO:0070956] (biological process) Relationships: is a type of regulation of neutrophil mediated killing of bacterium [GO:0070950]; is a type of GO:0070955; negatively regulates neutrophil-mediated killing of bacterium [GO:0070944] Sources: GOC:add, GOC:mah Subtypes: negative regulation of neutrophil mediated killing of gram-negative bacterium [GO:0070957], negative regulation of neutrophil mediated killing of gram-positive bacterium [GO:0070958] Definition: Any process that decreases the frequency, rate or extent of the directed killing of a bacterium by a neutrophil. Also known as: down regulation of neutrophil mediated killing of bacterium, down-regulation of neutrophil mediated killing of bacterium, downregulation of neutrophil mediated killing of bacterium, inhibition of neutrophil mediated killing of bacterium